holo-[acyl-carrier-protein] synthase activity [GO:0008897] (molecular function) Definition: Catalysis of the reaction: CoA + substrate-serine = adenosine 3',5'-bisphosphate + substrate-serine-4'-phosphopantetheine. The transfer of the 4'-phosphopantetheine (Ppant) co-factor from coenzyme A to the hydroxyl side chain of the serine residue of acyl- or peptidyl-carrier protein (ACP or PCP) to convert them from the apo to the holo form. References: PMID:10320345, PMID:11867633, PMID:8939709 Sources: EC:2.7.8.7 Also known as: 4'-phosphopantetheinyltransferase activity, alpha-aminoadipate reductase phosphopantetheinyl transferase activity, phosphopantetheinyltransferase activity, L-aminoadipate-semialdehyde dehydrogenase-phosphopantetheinyl transferase activity, holo-[peptidyl-carrier protein] synthase activity, 4'-phosphopantetheinyl transferase activity, ACPS activity, AcpS, CoA-[4'-phosphopantetheine]:apo-acyl-carrier-protein 4'-pantetheinephosphotransferase activity, CoA:apo-acyl-carrier-protein pantetheinephosphotransferase activity, P-pant transferase activity, PPTase activity, acyl carrier protein holoprotein (holo-ACP) synthetase activity, acyl carrier protein synthase activity, acyl carrier protein synthetase activity, alpha-aminoadipic semialdehyde dehydrogenase-phosphopantetheinyl transferase activity, alphaaminoadipic semialdehyde dehydrogenase-phosphopantetheinyl transferase activity, coenzyme A:fatty acid synthetase apoenzyme 4'-phosphopantetheine transferase activity, holo-ACP synthase activity, holo-ACP synthetase activity, holo-acyl-carrier-protein synthase activity, holosynthase activity, phosphopantetheinyl transferase Relationships: is a type of GO:0016780